negative regulation of laminaritriose transport [GO:1900304] (biological process) Also known as: down regulation of laminaritriose transport, down-regulation of laminaritriose transport, downregulation of laminaritriose transport, inhibition of laminaritriose transport Sources: GOC:TermGenie, GOC:mengo_curators Relationships: is a type of negative regulation of transport [GO:0051051]; is a type of regulation of laminaritriose transport [GO:1900303]; negatively regulates laminaritriose transport [GO:2001097] Definition: Any process that stops, prevents or reduces the frequency, rate or extent of laminaritriose transport.